{
  "term_id": "UNKNOWN:0003",
  "gene": "UniProtKB:Q9Y4F1",
  "gene_name": "FERM, ARHGEF and pleckstrin domain-containing protein 1",
  "gene_symbol": "FARP1",
  "term_label": "Unknown cellular component"
}